tyrosine 3-monooxygenase activator activity [GO:0036470] (molecular function) Also known as: TH activator activity, tyrosine hydroxylase activator activity Definition: Binds to and increases the activity of tyrosine 3-monooxygenase (tyrosine hydroxylase). Relationships: is a type of GO:0008047; positively regulates tyrosine 3-monooxygenase activity [GO:0004511] References: PMID:19703902 Sources: GOC:PARL, GOC:bf